{
  "term_label": "transcription coregulator activity",
  "gene_name": "Protein LYRIC",
  "term_id": "GO:0003712",
  "gene_symbol": "MTDH",
  "gene": "UniProtKB:Q86UE4"
}